{
  "gene": "UniProtKB:Q6ZWJ8",
  "gene_name": "Kielin_chordin-like protein",
  "term_label": "extracellular region",
  "gene_symbol": "KCP",
  "term_id": "GO:0005576"
}